response to hexane [GO:1901499] (biological process) Sources: GOC:TermGenie, GOC:mengo_curators Definition: Any process that results in a change in state or activity of a cell or an organism (in terms of movement, secretion, enzyme production, gene expression, etc.) as a result of a hexane stimulus. Relationships: is_a response to alkane [GO:1902778]